{
  "gene_name": "Gap junction alpha-3 protein",
  "gene": "UniProtKB:Q9Y6H8",
  "gene_symbol": "GJA3",
  "term_label": "cell-cell signaling",
  "term_id": "GO:0007267"
}